rough endoplasmic reticulum membrane [GO:0030867] (cellular component) Definition: The lipid bilayer surrounding the rough endoplasmic reticulum. Sources: GOC:mah Also known as: RER membrane, rough ER membrane Relationships: is a type of endoplasmic reticulum membrane [GO:0005789]; is a type of bounding membrane of organelle [GO:0098588]; BFO_0000050 rough endoplasmic reticulum [GO:0005791]